{
  "term_id": "GO:0003714",
  "gene_symbol": "PHF24",
  "gene": "UniProtKB:Q9UPV7",
  "term_label": "transcription corepressor activity",
  "gene_name": "PHD finger protein 24"
}